{
  "gene_symbol": "DCX",
  "gene": "UniProtKB:O43602",
  "gene_name": "Neuronal migration protein doublecortin",
  "term_label": "Unknown molecular function",
  "term_id": "UNKNOWN:0001"
}